{
  "gene": "UniProtKB:Q9C0G0",
  "term_label": "nucleus",
  "term_id": "GO:0005634",
  "gene_symbol": "ZNF407",
  "gene_name": "Zinc finger protein 407"
}